Ire1 complex [GO:1990332] (CC) References: PMID:18191223, PMID:25437541 Sources: GOC:bf, GOC:bhm Note: An example of this is Ire1 in S. cerevisiae (P32361) in PMID:18191223 (inferred from direct assay). Also known as: ER-bound kinase/endoribonuclease (RNase), inositol-requiring enzyme-1, IRE1 dimer, Ire1 complex dimer, Ire1 complex homodimer, Ire1 complex homooligomer, ERN1 complex Relationships: is a type of membrane protein complex [GO:0098796]; is a type of GO:0140534; is a type of GO:1902554; is a type of endoribonuclease complex [GO:1902555]; is part of GO:0005789 Definition: A type-I transmembrane protein complex located in the endoplasmic reticulum (ER) consisting of an IRE1-IRE1 dimer, which forms in response to the accumulation of unfolded protein in the ER. The dimeric complex has endoribonuclease (RNase) activity and evokes the unfolded protein response (UPR) by cleaving an intron of a mRNA coding for the transcription factor HAC1 in yeast or XBP1 in mammals; the complex cleaves a single phosphodiester bond in each of two RNA hairpins (with non-specific base paired stems and loops of consensus sequence CNCNNGN, where N is any base) to remove an intervening intron from the target transcript.